{
  "gene": "UniProtKB:O14960",
  "gene_symbol": "LECT2",
  "term_label": "Unknown biological process",
  "term_id": "UNKNOWN:0002",
  "gene_name": "Leukocyte cell-derived chemotaxin-2"
}